{
  "term_label": "extracellular space",
  "gene_symbol": "CER1",
  "gene": "UniProtKB:O95813",
  "term_id": "GO:0005615",
  "gene_name": "Cerberus"
}